{
  "gene": "UniProtKB:Q13576",
  "term_id": "GO:0051015",
  "gene_name": "Ras GTPase-activating-like protein IQGAP2",
  "gene_symbol": "IQGAP2",
  "term_label": "actin filament binding"
}